cortisol O-acetyltransferase activity [GO:0047784] (molecular function) Relationships: is a type of O-acetyltransferase activity [GO:0016413] Also known as: acetyl-CoA:cortisol O-acetyltransferase activity, corticosteroid acetyltransferase activity, corticosteroid-21-O-acetyltransferase activity, cortisol acetyltransferase activity Definition: Catalysis of the reaction: acetyl-CoA + cortisol = CoA + cortisol 21-acetate. Sources: EC:2.3.1.27, RHEA:17073